ATP-independent citrate lyase complex [GO:0009346] (cellular component) Definition: Citrate lyase is a multienzyme complex with three constituents: the alpha subunit, citrate-ACP transferase; the beta subunit, citryl-ACP lyase; and the gamma subunit, an acyl-carrier protein which also carries the prosthetic group components. All three subunits are required for citrate lyase enzyme activity. This enzyme has only been found in bacteria. Note: Note that this complex has only been found in bacteria. For eukaryotic cytrate lyases, consider GO:0140615 ; ATP-dependent citrate lyase complex. Relationships: is a type of intracellular protein-containing complex [GO:0140535]; is a type of catalytic complex [GO:1902494] References: PMID:32302313 Also known as: citrate lyase complex, citrate synthase complex